phenylglyoxylate dehydrogenase (acylating) activity [GO:0047110] (MF) Relationships: is a type of oxidoreductase activity, acting on the aldehyde or oxo group of donors, NAD or NADP as acceptor [GO:0016620] Definition: Catalysis of the reaction: CoA + NAD+ + phenylglyoxylate = benzoyl-CoA + CO2 + NADH. Sources: RHEA:10372 Also known as: phenylglyoxylate:NAD+ oxidoreductase activity